UDP-N-acetylglucosamine 2-epimerase activity [GO:0008761] (molecular function) Relationships: is a type of racemase and epimerase activity, acting on carbohydrates and derivatives [GO:0016857] Sources: EC:5.1.3.14 Also known as: UDP-GlcNAc-2-epimerase activity, UDP-N-acetyl-D-glucosamine 2-epimerase activity, UDP-N-acetylglucosamine 2'-epimerase activity, uridine diphosphate-N-acetylglucosamine-2'-epimerase activity, uridine diphospho-N-acetylglucosamine 2'-epimerase activity, uridine diphosphoacetylglucosamine 2'-epimerase activity Definition: Catalysis of the reaction: UDP-N-acetyl-D-glucosamine = UDP-N-acetyl-D-mannosamine.